{
  "gene_name": "Ubiquitin-like protein 7",
  "term_label": "cytosol",
  "term_id": "GO:0005829",
  "gene_symbol": "UBL7",
  "gene": "UniProtKB:Q96S82"
}